{
  "gene_symbol": "GPATCH1",
  "term_id": "GO:0003723",
  "gene_name": "G patch domain-containing protein 1",
  "term_label": "RNA binding",
  "gene": "UniProtKB:Q9BRR8"
}